{
  "term_id": "UNKNOWN:0002",
  "gene_name": "Olfactory receptor 5H2",
  "gene": "UniProtKB:Q8NGV7",
  "gene_symbol": "OR5H2",
  "term_label": "Unknown biological process"
}